{
  "gene_symbol": "UNC5A",
  "term_label": "anterior/posterior axon guidance",
  "gene_name": "Netrin receptor UNC5A",
  "term_id": "GO:0033564",
  "gene": "UniProtKB:Q6ZN44"
}